{
  "gene": "UniProtKB:Q9Y277",
  "gene_symbol": "VDAC3",
  "gene_name": "Voltage-dependent anion-selective channel protein 3",
  "term_label": "voltage-gated monoatomic anion channel activity",
  "term_id": "GO:0008308"
}